{
  "term_id": "GO:0005525",
  "term_label": "GTP binding",
  "gene_name": "Rho-related GTP-binding protein RhoC",
  "gene_symbol": "RHOC",
  "gene": "UniProtKB:P08134"
}